{
  "gene_symbol": "MELK",
  "term_id": "GO:0004715",
  "gene_name": "Maternal embryonic leucine zipper kinase",
  "term_label": "non-membrane spanning protein tyrosine kinase activity",
  "gene": "UniProtKB:Q14680"
}